DNA damage sensor activity [GO:0140612] (molecular function) Subtypes: GO:0140664 Also known as: DNA damage sensing activity References: PMID:31995034 Definition: A molecule that recognises toxic DNA structures, for example, double-strand breaks or collapsed replication forks, and initiates a signaling response. Relationships: is a type of molecular sensor activity [GO:0140299]; has part damaged DNA binding [GO:0003684]